glomerular epithelium development [GO:0072010] (biological process) Definition: The process whose specific outcome is the progression of the glomerular epithelium over time, from its formation to the mature structure. The glomerular epithelium is an epithelial tissue that covers the outer surfaces of the glomerulus. The glomerular epithelium consists of both parietal and visceral epithelium. Metanephric glomerular parietal epithelial cells are specialized epithelial cells that form tight junctions as a barrier to protein transport. A metanephric glomerular visceral epithelial cell is a specialized epithelial cell that contains 'feet' that interdigitate with the 'feet' of other glomerular epithelial cells in the metanephros. Sources: GOC:mtg_kidney_jan10 Subtypes: mesonephric glomerular epithelium development [GO:0061232], glomerular endothelium development [GO:0072011], GO:0072244 Relationships: is a type of GO:0072009; is part of glomerulus development [GO:0032835]